{
  "gene_symbol": "HIP1R",
  "term_id": "GO:0045742",
  "gene": "UniProtKB:O75146",
  "gene_name": "Huntingtin-interacting protein 1-related protein",
  "term_label": "positive regulation of epidermal growth factor receptor signaling pathway"
}